{
  "gene_symbol": "SH3RF1",
  "term_id": "GO:0061630",
  "term_label": "ubiquitin protein ligase activity",
  "gene": "UniProtKB:Q7Z6J0",
  "gene_name": "E3 ubiquitin-protein ligase SH3RF1"
}